regulation of lactose biosynthetic process [GO:1903534] (biological process) Definition: Any process that modulates the frequency, rate or extent of lactose biosynthetic process. Also known as: regulation of lactose anabolism, regulation of lactose biosynthesis, regulation of lactose formation, regulation of lactose synthesis References: PMID:12018418 Sources: GOC:TermGenie, GOC:mr, GO_REF:0000058 Relationships: is a type of regulation of carbohydrate biosynthetic process [GO:0043255]; regulates lactose biosynthetic process [GO:0005989] Subtypes: GO:1903535, positive regulation of lactose biosynthetic process [GO:1903536]